{
  "term_id": "GO:0005615",
  "term_label": "extracellular space",
  "gene": "UniProtKB:Q8IUL8",
  "gene_symbol": "CILP2",
  "gene_name": "Cartilage intermediate layer protein 2"
}